apelin receptor binding [GO:0031704] (molecular function) Definition: Binding to an apelin receptor. Also known as: APJ receptor binding, apelin receptor ligand Relationships: is a type of neuropeptide receptor binding [GO:0071855] References: PMID:12787050 Sources: GOC:mah, GOC:nln, GOC:vp